{
  "term_label": "cellular response to ionizing radiation",
  "gene": "UniProtKB:Q6WBX8",
  "gene_symbol": "RAD9B",
  "gene_name": "Cell cycle checkpoint control protein RAD9B",
  "term_id": "GO:0071479"
}